{
  "gene_name": "TLC domain-containing protein 1",
  "gene": "UniProtKB:Q96CP7",
  "gene_symbol": "TLCD1",
  "term_id": "GO:0055091",
  "term_label": "phospholipid homeostasis"
}